{
  "term_id": "GO:0006096",
  "gene": "UniProtKB:P30613",
  "gene_symbol": "PKLR",
  "term_label": "glycolytic process",
  "gene_name": "Pyruvate kinase PKLR"
}